RNA nuclear export complex [GO:0042565] (cellular component) References: PMID:9323123 Sources: GOC:jl Relationships: is a type of nucleocytoplasmic transport complex [GO:0031074] Definition: A complex which usually consists of three components, e.g. in Xenopus and yeast, the export receptor CRM1 (also known as exportin 1), the Ran protein and any RNA with a nuclear export sequence (NES). The complex acts to export RNA molecules with a NES from the nucleus through a nuclear pore.